postsynaptic density, intracellular component [GO:0099092] (cellular component) Definition: A network of proteins adjacent to the postsynaptic membrane forming an electron dense disc. Its major components include neurotransmitter receptors and the proteins that spatially and functionally organize neurotransmitter receptors in the adjacent membrane, such as anchoring and scaffolding molecules, signaling enzymes and cytoskeletal components. Relationships: is a type of GO:0099091; is part of postsynaptic density [GO:0014069] Sources: GOC:dos